regulation of protein K48-linked deubiquitination [GO:1903093] (biological process) Relationships: is a type of regulation of protein deubiquitination [GO:0090085]; regulates GO:0071108 Sources: GOC:PARL, GOC:TermGenie, GOC:bf, GO_REF:0000058 Subtypes: GO:1903094 Definition: Any process that modulates the frequency, rate or extent of protein K48-linked deubiquitination.